{
  "term_id": "GO:0005615",
  "gene_name": "Sulfhydryl oxidase 2",
  "gene": "UniProtKB:Q6ZRP7",
  "gene_symbol": "QSOX2",
  "term_label": "extracellular space"
}